{
  "term_label": "kinocilium",
  "gene_name": "Stereocilin",
  "term_id": "GO:0060091",
  "gene": "UniProtKB:Q7RTU9",
  "gene_symbol": "STRC"
}